{
  "gene_symbol": "SEMA4B",
  "gene_name": "Semaphorin-4B",
  "gene": "UniProtKB:Q9NPR2",
  "term_id": "GO:0071526",
  "term_label": "semaphorin-plexin signaling pathway"
}